{
  "gene_symbol": "HNRNPU",
  "gene_name": "Heterogeneous nuclear ribonucleoprotein U",
  "term_label": "alternative mRNA splicing, via spliceosome",
  "term_id": "GO:0000380",
  "gene": "UniProtKB:Q00839"
}